{
  "gene_symbol": "NRCAM",
  "gene": "UniProtKB:Q92823",
  "term_id": "GO:0098632",
  "term_label": "cell-cell adhesion mediator activity",
  "gene_name": "Neuronal cell adhesion molecule"
}